{
  "gene_symbol": "LPAR2",
  "gene": "UniProtKB:Q9HBW0",
  "term_label": "adenylate cyclase-activating G protein-coupled receptor signaling pathway",
  "gene_name": "Lysophosphatidic acid receptor 2",
  "term_id": "GO:0007189"
}